{
  "term_label": "Unknown molecular function",
  "gene": "UniProtKB:Q5SZK8",
  "term_id": "UNKNOWN:0001",
  "gene_symbol": "FREM2",
  "gene_name": "FRAS1-related extracellular matrix protein 2"
}